{
  "gene_name": "Ankyrin repeat domain-containing protein 18B",
  "term_label": "Unknown molecular function",
  "gene_symbol": "ANKRD18B",
  "gene": "UniProtKB:A2A2Z9",
  "term_id": "UNKNOWN:0001"
}